{
  "term_id": "GO:0017022",
  "gene": "UniProtKB:Q8NFW9",
  "gene_name": "Rab effector MyRIP",
  "gene_symbol": "MYRIP",
  "term_label": "myosin binding"
}